{
  "term_id": "GO:0006508",
  "gene": "UniProtKB:Q9HC96",
  "gene_symbol": "CAPN10",
  "gene_name": "Calpain-10",
  "term_label": "proteolysis"
}